{
  "gene": "UniProtKB:Q8NFJ5",
  "gene_name": "Retinoic acid-induced protein 3",
  "gene_symbol": "GPRC5A",
  "term_id": "UNKNOWN:0002",
  "term_label": "Unknown biological process"
}